{
  "term_id": "GO:0022857",
  "gene": "UniProtKB:Q96NB2",
  "gene_name": "Sideroflexin-2",
  "gene_symbol": "SFXN2",
  "term_label": "transmembrane transporter activity"
}